positive regulation of Lewy body formation [GO:0140124] (biological process) Definition: Any process that activates or increases the frequency, rate or extent of Lewy body formation. Sources: GOC:sl Relationships: is a type of positive regulation of inclusion body assembly [GO:0090261]; is a type of GO:0140122; positively regulates Lewy body formation [GO:0140121]